{
  "term_label": "TRAIL-activated apoptotic signaling pathway",
  "gene_symbol": "TNFRSF10C",
  "term_id": "GO:0036462",
  "gene": "UniProtKB:O14798",
  "gene_name": "Tumor necrosis factor receptor superfamily member 10C"
}